positive regulation of D-glucose import [GO:0046326] (biological process) Definition: Any process that activates or increases the frequency, rate or extent of the import of the hexose monosaccharide glucose into a cell or organelle. Relationships: is a type of positive regulation of D-glucose transmembrane transport [GO:0010828]; is a type of regulation of D-glucose import [GO:0046324]; positively regulates D-glucose import [GO:0046323] Also known as: positive regulation of glucose import, positive regulation of glucose uptake, up regulation of glucose import, up-regulation of glucose import, upregulation of glucose import, activation of glucose import, stimulation of glucose import Sources: GOC:ai, GOC:dph, GOC:tb